{
  "term_label": "extracellular space",
  "gene": "UniProtKB:P0DTE7",
  "gene_name": "Alpha-amylase 1B",
  "term_id": "GO:0005615",
  "gene_symbol": "AMY1B"
}